{
  "term_label": "tRNA-splicing ligase complex",
  "term_id": "GO:0072669",
  "gene": "UniProtKB:Q52LJ0",
  "gene_name": "Protein FAM98B",
  "gene_symbol": "FAM98B"
}